{
  "gene_name": "Max dimerization protein 3",
  "gene_symbol": "MXD3",
  "term_label": "regulation of transcription by RNA polymerase II",
  "term_id": "GO:0006357",
  "gene": "UniProtKB:Q9BW11"
}